{
  "gene_symbol": "SNX16",
  "gene": "UniProtKB:P57768",
  "gene_name": "Sorting nexin-16",
  "term_label": "early endosome",
  "term_id": "GO:0005769"
}